{
  "gene_name": "Integrin alpha-1",
  "gene_symbol": "ITGA1",
  "gene": "UniProtKB:P56199",
  "term_label": "cell-cell adhesion",
  "term_id": "GO:0098609"
}